{
  "term_label": "negative regulation of microglial cell activation",
  "gene": "UniProtKB:Q7Z5A8",
  "gene_symbol": "TAFA3",
  "gene_name": "Chemokine-like protein TAFA-3",
  "term_id": "GO:1903979"
}